guanine/thymine mispair binding [GO:0032137] (molecular function) Sources: GOC:vk Definition: Binding to a double-stranded DNA region containing a G/T mispair. Relationships: is a type of mismatched DNA binding [GO:0030983] Also known as: G/T mispair binding, T/G mispair binding, thymine/guanine mispair binding